{
  "term_label": "Unknown molecular function",
  "gene_name": "Protein SGT1 homolog",
  "gene": "UniProtKB:Q9Y2Z0",
  "term_id": "UNKNOWN:0001",
  "gene_symbol": "SUGT1"
}